regulation of chylomicron remodeling [GO:0090318] (biological process) Definition: Any process that modulates the rate, frequency, or extent of chylomicron remodeling. Chylomicron remodeling is the acquisition, loss or modification of a protein or lipid within a chylomicron, including the hydrolysis of triglyceride by lipoprotein lipase and the subsequent loss of free fatty acid. Sources: GOC:tb Also known as: regulation of chylomicron remodelling Relationships: is a type of regulation of cellular component organization [GO:0051128]; is a type of GO:0051239; regulates chylomicron remodeling [GO:0034371] Subtypes: GO:0090319